{
  "gene_symbol": "TMEM102",
  "gene": "UniProtKB:Q8N9M5",
  "gene_name": "Transmembrane protein 102",
  "term_label": "Unknown biological process",
  "term_id": "UNKNOWN:0002"
}